{
  "term_id": "GO:0060070",
  "term_label": "canonical Wnt signaling pathway",
  "gene_symbol": "WNT3",
  "gene_name": "Proto-oncogene Wnt-3",
  "gene": "UniProtKB:P56703"
}